{
  "gene_name": "Putative protein MSS51 homolog, mitochondrial",
  "term_label": "Unknown molecular function",
  "gene_symbol": "MSS51",
  "gene": "UniProtKB:Q4VC12",
  "term_id": "UNKNOWN:0001"
}